circulatory system process [GO:0003013] (biological process) Relationships: is a type of GO:0003008 Definition: An organ system process carried out by any of the organs or tissues of the circulatory system. The circulatory system is an organ system that moves extracellular fluids to and from tissue within a multicellular organism. Sources: GOC:mtg_cardio Subtypes: heart process [GO:0003015], GO:0003017, vascular process in circulatory system [GO:0003018], blood circulation [GO:0008015], GO:1990029